{
  "gene": "UniProtKB:Q9BR61",
  "term_id": "UNKNOWN:0002",
  "gene_name": "Acyl-CoA-binding domain-containing protein 6",
  "gene_symbol": "ACBD6",
  "term_label": "Unknown biological process"
}